negative regulation of mesenchymal cell apoptotic process [GO:2001054] (biological process) Definition: Any process that stops, prevents or reduces the frequency, rate or extent of mesenchymal cell apoptotic process. Sources: GOC:mtg_apoptosis, GOC:obol Also known as: negative regulation of mesenchymal cell apoptosis Relationships: is_a negative regulation of apoptotic process [GO:0043066]; is a type of regulation of mesenchymal cell apoptotic process [GO:2001053]; negatively regulates mesenchymal cell apoptotic process [GO:0097152] Subtypes: negative regulation of mesenchymal cell apoptotic process involved in nephron morphogenesis [GO:0072040], negative regulation of mesenchymal cell apoptotic process involved in metanephros development [GO:1900212]